protein localization to mitochondrion [GO:0070585] (biological process) Relationships: is a type of protein localization to organelle [GO:0033365] Sources: GOC:ecd Subtypes: protein import into mitochondrial matrix [GO:0030150], protein import into mitochondrial intermembrane space [GO:0045041] Definition: A process in which a protein is transported to, or maintained in, a location within the mitochondrion. Also known as: protein localisation in mitochondrion, protein localization in mitochondrion